{
  "gene_name": "Talin-1",
  "term_id": "GO:0005925",
  "gene": "UniProtKB:Q9Y490",
  "gene_symbol": "TLN1",
  "term_label": "focal adhesion"
}